{
  "gene": "UniProtKB:Q9H9Y2",
  "gene_symbol": "RPF1",
  "term_id": "UNKNOWN:0001",
  "gene_name": "Ribosome production factor 1",
  "term_label": "Unknown molecular function"
}